regulation of non-canonical NF-kappaB signal transduction [GO:1901222] (biological process) Also known as: regulation of NIK/NF-kappaB cascade, regulation of NIK/NF-kappaB signaling, regulation of non-canonical NF-KB signaling, regulation of noncanonical NF-kappaB signaling, regulation of noncanonical nuclear factor kappaB (NF-kappaB) pathway, NF-KB import into nucleus, NF-kappaB import into nucleus, regulation of NF-kappaB import into nucleus, regulation of p52-dependent NF-kappaB signaling Sources: GOC:TermGenie Relationships: is a type of GO:1902531; regulates non-canonical NF-kappaB signal transduction [GO:0038061] Definition: Any process that modulates the frequency, rate or extent of the non-canonical NF-kappaB signaling cascade. Subtypes: GO:1901223, positive regulation of non-canonical NF-kappaB signal transduction [GO:1901224]